{
  "gene_name": "Cullin-2",
  "term_label": "SCF-dependent proteasomal ubiquitin-dependent protein catabolic process",
  "gene": "UniProtKB:Q13617",
  "gene_symbol": "CUL2",
  "term_id": "GO:0031146"
}